{
  "term_id": "GO:0000976",
  "gene": "UniProtKB:Q14865",
  "gene_symbol": "ARID5B",
  "gene_name": "AT-rich interactive domain-containing protein 5B",
  "term_label": "transcription cis-regulatory region binding"
}